{
  "term_label": "Unknown molecular function",
  "gene_name": "Uncharacterized protein FAM167A-AS1",
  "gene_symbol": "FAM167A-AS1",
  "gene": "UniProtKB:Q96KT0",
  "term_id": "UNKNOWN:0001"
}